protein-N(PI)-phosphohistidine-N-acetylgalactosamine phosphotransferase system transporter activity [GO:0022881] (MF) Sources: GOC:mtg_transport, ISBN:0815340729 Also known as: N-acetylgalactosamine PTS transporter activity Relationships: is a type of protein-N(PI)-phosphohistidine-sugar phosphotransferase activity [GO:0008982]; is a type of GO:0015571; is a type of D-glucose transmembrane transporter activity [GO:0055056] Definition: Catalysis of the PEP-dependent, phosphoryl transfer-driven transport of substances across a membrane. The transport happens by catalysis of the reaction: protein N-phosphohistidine + N-acetylgalactosamine(out) = protein histidine + N-acetylgalactosamine phosphate(in). This differs from primary and secondary active transport in that the solute is modified during transport.